{
  "gene_name": "Zona pellucida-binding protein 2",
  "term_label": "Unknown molecular function",
  "gene": "UniProtKB:Q6X784",
  "gene_symbol": "ZPBP2",
  "term_id": "UNKNOWN:0001"
}